{
  "gene_name": "Transmembrane protein 248",
  "gene_symbol": "TMEM248",
  "term_id": "UNKNOWN:0002",
  "term_label": "Unknown biological process",
  "gene": "UniProtKB:Q9NWD8"
}